{
  "gene_symbol": "KLHL33",
  "term_id": "UNKNOWN:0002",
  "gene_name": "Kelch-like protein 33",
  "term_label": "Unknown biological process",
  "gene": "UniProtKB:A6NCF5"
}